{
  "gene_name": "Protein BEX4",
  "term_id": "UNKNOWN:0002",
  "gene_symbol": "BEX4",
  "gene": "UniProtKB:Q9NWD9",
  "term_label": "Unknown biological process"
}